postsynaptic cytoskeleton [GO:0099571] (cellular component) Definition: The portion of the cytoskeleton contained within the postsynapse. Subtypes: GO:0098836, postsynaptic actin cytoskeleton [GO:0098871], postsynaptic intermediate filament cytoskeleton [GO:0099160], GO:0099189, postsynaptic septin cytoskeleton [GO:0150050] References: PMID:19889835 Sources: GOC:dos Relationships: is_a cytoskeleton [GO:0005856]; is part of postsynapse [GO:0098794]